{
  "term_label": "nervous system development",
  "gene_name": "RNA binding protein fox-1 homolog 1",
  "term_id": "GO:0007399",
  "gene": "UniProtKB:Q9NWB1",
  "gene_symbol": "RBFOX1"
}